voltage-gated chloride channel activity [GO:0005247] (molecular function) Subtypes: organellar voltage-gated chloride channel activity [GO:0015274] Regulation: positively regulated by GO:1902943 Also known as: voltage gated chloride channel activity, voltage-dependent chloride channel activity Relationships: is a type of GO:0005254; is_a voltage-gated monoatomic anion channel activity [GO:0008308] Definition: Enables the transmembrane transfer of a chloride ion by a voltage-gated channel. A voltage-gated channel is a channel whose open state is dependent on the voltage across the membrane in which it is embedded. Sources: GOC:mtg_transport, ISBN:0815340729